{
  "gene": "UniProtKB:P62324",
  "gene_name": "Protein BTG1",
  "term_label": "nucleus",
  "gene_symbol": "BTG1",
  "term_id": "GO:0005634"
}